{
  "term_label": "Unknown molecular function",
  "gene_symbol": "ADARB2-AS1",
  "gene_name": "Putative uncharacterized protein ADARB2-AS1",
  "term_id": "UNKNOWN:0001",
  "gene": "UniProtKB:A8MUL3"
}